{
  "term_id": "UNKNOWN:0002",
  "term_label": "Unknown biological process",
  "gene_name": "A-kinase anchor protein SPHKAP",
  "gene": "UniProtKB:Q2M3C7",
  "gene_symbol": "SPHKAP"
}